inosine kinase activity [GO:0008906] (molecular function) Definition: Catalysis of the reaction: ATP + inosine = ADP + IMP. Sources: EC:2.7.1.73 Also known as: ATP:inosine 5'-phosphotransferase activity, inosine kinase (phosphorylating), inosine-guanosine kinase activity Relationships: is a type of kinase activity [GO:0016301]; is a type of phosphotransferase activity, alcohol group as acceptor [GO:0016773]